cortical granule exocytosis [GO:0060471] (biological process) Definition: The process of secretion by a cell that results in the release of intracellular molecules contained within a cortical granule by fusion of the vesicle with the plasma membrane of a cell. A cortical granule is a specialized secretory vesicle that is released during egg activation that changes the surface of the egg to prevent polyspermy. Relationships: is a type of calcium-ion regulated exocytosis [GO:0017156]; is part of GO:0060468 Also known as: cortical granule release, cortical reaction Sources: GOC:dph Regulation: positively regulated by positive regulation of cortical granule exocytosis by positive regulation of cytosolic calcium ion concentration [GO:0060472]